{
  "gene_symbol": "RAP1GAP2",
  "gene_name": "Rap1 GTPase-activating protein 2",
  "term_label": "GTPase activator activity",
  "term_id": "GO:0005096",
  "gene": "UniProtKB:Q684P5"
}